{
  "gene_symbol": "RCHY1",
  "gene": "UniProtKB:Q96PM5",
  "term_id": "GO:0005634",
  "gene_name": "RING finger and CHY zinc finger domain-containing protein 1",
  "term_label": "nucleus"
}